establishment of animal organ orientation [GO:0048561] (biological process) Sources: GOC:jid Definition: The process that determines the orientation of an animal organ or tissue with reference to an axis. Relationships: is a type of GO:0048560; BFO_0000050 GO:0009887